{
  "gene_name": "Transmembrane emp24 domain-containing protein 5",
  "term_label": "COPII-coated ER to Golgi transport vesicle",
  "term_id": "GO:0030134",
  "gene": "UniProtKB:Q9Y3A6",
  "gene_symbol": "TMED5"
}